{
  "gene_name": "Uncharacterized protein C11orf71",
  "gene_symbol": "C11orf71",
  "term_label": "Unknown cellular component",
  "term_id": "UNKNOWN:0003",
  "gene": "UniProtKB:Q6IPW1"
}